somatic stem cell division [GO:0048103] (biological process) Definition: The self-renewing division of a somatic stem cell, a stem cell that can give rise to cell types of the body other than those of the germ-line. Also known as: somatic stem cell renewal Sources: GOC:jid, ISBN:0582227089 Regulation: regulated by GO:1904675; negatively regulated by negative regulation of somatic stem cell division [GO:1904676]; positively regulated by positive regulation of somatic stem cell division [GO:1904677] Subtypes: skeletal muscle satellite stem cell asymmetric division [GO:0014833], neuronal stem cell division [GO:0036445], symmetric division of skeletal muscle satellite stem cell [GO:0098726] Relationships: is a type of stem cell division [GO:0017145]